{
  "term_id": "GO:0000981",
  "gene_symbol": "ELF2",
  "gene_name": "ETS-related transcription factor Elf-2",
  "term_label": "DNA-binding transcription factor activity, RNA polymerase II-specific",
  "gene": "UniProtKB:Q15723"
}